{
  "term_id": "GO:0005634",
  "gene": "UniProtKB:Q9NWZ3",
  "gene_symbol": "IRAK4",
  "term_label": "nucleus",
  "gene_name": "Interleukin-1 receptor-associated kinase 4"
}